{
  "gene": "UniProtKB:Q8TF50",
  "term_label": "Unknown cellular component",
  "term_id": "UNKNOWN:0003",
  "gene_name": "Zinc finger protein 526",
  "gene_symbol": "ZNF526"
}